{
  "term_label": "nucleus",
  "gene_name": "Zinc finger protein 799",
  "gene_symbol": "ZNF799",
  "term_id": "GO:0005634",
  "gene": "UniProtKB:Q96GE5"
}